{
  "gene_symbol": "FGF13",
  "gene": "UniProtKB:Q92913",
  "term_id": "GO:0005737",
  "term_label": "cytoplasm",
  "gene_name": "Fibroblast growth factor 13"
}